{
  "gene_symbol": "ZNF850",
  "term_label": "regulation of transcription by RNA polymerase II",
  "gene_name": "Zinc finger protein 850",
  "term_id": "GO:0006357",
  "gene": "UniProtKB:A8MQ14"
}